{
  "gene_name": "Lysine-specific demethylase 7A",
  "gene": "UniProtKB:Q6ZMT4",
  "gene_symbol": "KDM7A",
  "term_label": "regulation of transcription by RNA polymerase II",
  "term_id": "GO:0006357"
}